negative regulation of osteoblast proliferation [GO:0033689] (biological process) Also known as: down regulation of osteoblast proliferation, down-regulation of osteoblast proliferation, downregulation of osteoblast proliferation, inhibition of osteoblast proliferation Definition: Any process that stops, prevents or reduces the rate or extent of osteoblast proliferation. Relationships: is a type of GO:0008285; is a type of regulation of osteoblast proliferation [GO:0033688]; negatively regulates osteoblast proliferation [GO:0033687] Sources: GOC:mah